positive regulation of canonical Wnt signaling pathway [GO:0090263] (biological process) Sources: GOC:tb Definition: Any process that increases the rate, frequency, or extent of the Wnt signaling pathway through beta-catenin, the series of molecular signals initiated by binding of a Wnt protein to a frizzled family receptor on the surface of the target cell, followed by propagation of the signal via beta-catenin, and ending with a change in transcription of target genes. Also known as: positive regulation of Wnt receptor signaling pathway through beta-catenin, positive regulation of canonical Wnt receptor signaling pathway, positive regulation of canonical Wnt receptor signalling pathway, positive regulation of canonical Wnt-activated signaling pathway, positive regulation of catenin import into nucleus, positive regulation of catenin protein nuclear translocation Relationships: is a type of positive regulation of Wnt signaling pathway [GO:0030177]; is a type of regulation of canonical Wnt signaling pathway [GO:0060828]; positively regulates canonical Wnt signaling pathway [GO:0060070]